modulation by host of viral exo-alpha-sialidase activity [GO:0044866] (biological process) Definition: The process in which a host organism effects a change in viral exo-alpha-sialidase activity, the catalysis of the hydrolysis of peptide bonds in a protein. Sources: GOC:jl Relationships: is a type of modulation by host of viral catalytic activity [GO:0044867]; regulates GO:0004308